mitotic S phase [GO:0000084] (biological process) Also known as: S phase of mitotic cell cycle, S-phase of mitotic cell cycle Note: Note that this term should not be used for direct annotation. If you are trying to make an annotation to x phase, it is likely that the correct annotation is 'regulation of x/y phase transition' or to a process which occurs during the reported phase (i.e mitotic DNA replication for mitotic S-phase). To capture the phase when a specific location or process is observed, the phase term can be used in an annotation extension (PMID:24885854) applied to a cellular component term (with the relation exists_during) or a biological process term (with the relation happens_during). Sources: GOC:mtg_cell_cycle Relationships: is a type of S phase [GO:0051320]; is part of mitotic interphase [GO:0051329] Definition: The cell cycle phase, following G1, during which DNA synthesis takes place as part of a mitotic cell cycle.